protein localization to nucleolar rDNA repeats [GO:0034503] (biological process) Sources: GOC:mah Definition: Any process in which a protein is transported to, or maintained at, the rDNA repeats on a chromosome in the nucleolus. Also known as: protein localisation to nucleolar rDNA repeats, condensin localization to nucleolar rDNA repeats Relationships: is a type of protein localization to chromosome [GO:0034502]; is part of nucleolus organization [GO:0007000]